ER-nucleus signaling pathway [GO:0006984] (biological process) Also known as: ER to nucleus signaling pathway, ER to nucleus signalling pathway, ER-nuclear signaling pathway, ER-nuclear signalling pathway, endoplasmic reticulum to nucleus signaling pathway, endoplasmic reticulum-nuclear signaling pathway Relationships: is a type of intracellular signal transduction [GO:0035556] Definition: The series of molecular signals that conveys information from the endoplasmic reticulum to the nucleus, usually resulting in a change in transcriptional regulation. Subtypes: ER overload response [GO:0006983], SREBP signaling pathway [GO:0032933], PERK-mediated unfolded protein response [GO:0036499], ATF6-mediated unfolded protein response [GO:0036500] Sources: GOC:mah